{
  "term_label": "heterotrimeric G-protein complex",
  "gene_symbol": "GNAI2",
  "gene_name": "Guanine nucleotide-binding protein G(i) subunit alpha-2",
  "gene": "UniProtKB:P04899",
  "term_id": "GO:0005834"
}